{
  "gene_name": "Meteorin-like protein",
  "term_label": "energy homeostasis",
  "gene_symbol": "METRNL",
  "gene": "UniProtKB:Q641Q3",
  "term_id": "GO:0097009"
}